D-fuconate dehydratase activity [GO:0047818] (molecular function) Relationships: is a type of hydro-lyase activity [GO:0016836] Definition: Catalysis of the reaction: D-fuconate = 2-dehydro-3-deoxy-D-fuconate + H2O. Sources: EC:4.2.1.67, RHEA:12949 Also known as: D-fuconate hydratase activity, D-fuconate hydro-lyase (2-dehydro-3-deoxy-D-fuconate-forming), D-fuconate hydro-lyase activity